regulation of cytoplasmic translational initiation in response to stress [GO:1990611] (biological process) Definition: Modulation of the frequency, rate or extent of cytoplasmic translational initiation as a result of a stimulus indicating the organism is under stress. The stress is usually, but not necessarily, exogenous (e.g. temperature, humidity, ionizing radiation). References: PMID:16278445 Subtypes: negative regulation of cytoplasmic translational initiation in response to stress [GO:1990625] Relationships: is a type of regulation of translational initiation in response to stress [GO:0043558]; is_a regulation of cytoplasmic translational initiation [GO:1904688]; is a type of GO:1990497